{
  "term_label": "Unknown cellular component",
  "gene_name": "T cell receptor gamma joining 2 (Fragment)",
  "gene": "UniProtKB:A0A5H1ZRR4",
  "term_id": "UNKNOWN:0003",
  "gene_symbol": "TRGJ2"
}